tRNA (cytidine(32)/uridine(32)-2'-O)-methyltransferase activity [GO:0160206] (molecular function) Definition: Catalysis of the reaction: cytidine(32)/uridine(32) in tRNA + S-adenosyl-L-methionine = 2'-O-methylcytidine(32)/2'-O-methyluridine(32) in tRNA + H+ + S-adenosyl-L-homocysteine. Also known as: TrMet(Xm32) activity Sources: EC:2.1.1.200 Relationships: is a type of tRNA (uridine) methyltransferase activity [GO:0016300]; is a type of tRNA (cytidine) methyltransferase activity [GO:0016427]